{
  "term_label": "hormone activity",
  "term_id": "GO:0005179",
  "gene": "UniProtKB:P16860",
  "gene_symbol": "NPPB",
  "gene_name": "Natriuretic peptides B"
}